{
  "gene": "UniProtKB:Q9HBW1",
  "term_label": "postsynaptic density protein 95 clustering",
  "gene_name": "Leucine-rich repeat-containing protein 4",
  "term_id": "GO:0097119",
  "gene_symbol": "LRRC4"
}